{
  "gene": "UniProtKB:P32780",
  "term_label": "Unknown molecular function",
  "gene_name": "General transcription factor IIH subunit 1",
  "gene_symbol": "GTF2H1",
  "term_id": "UNKNOWN:0001"
}